{
  "gene_name": "Transcription factor SOX-21",
  "gene": "UniProtKB:Q9Y651",
  "gene_symbol": "SOX21",
  "term_label": "nucleus",
  "term_id": "GO:0005634"
}